{
  "gene": "UniProtKB:Q9Y547",
  "term_id": "UNKNOWN:0001",
  "gene_symbol": "IFT25",
  "gene_name": "Intraflagellar transport protein 25 homolog",
  "term_label": "Unknown molecular function"
}